{
  "term_label": "Unknown molecular function",
  "gene_symbol": "CRELD1",
  "gene": "UniProtKB:Q96HD1",
  "gene_name": "Protein disulfide isomerase CRELD1",
  "term_id": "UNKNOWN:0001"
}